CCU codon-amino acid adaptor activity [GO:0033421] (molecular function) Sources: GOC:mah Definition: A triplet codon-amino acid adaptor activity that recognizes a CCU codon. Relationships: is a type of triplet codon-amino acid adaptor activity [GO:0030533] Note: Note that in the standard genetic code, CCT codes for proline. Also known as: CCT codon-amino acid adaptor activity, proline tRNA